negative regulation of methane biosynthetic process from carbon monoxide [GO:1900337] (BP) Relationships: is a type of regulation of methane biosynthetic process from carbon monoxide [GO:1900336]; is a type of negative regulation of alkane biosynthetic process [GO:1901578]; is a type of GO:1901856; RO_0002212 methane biosynthetic process from carbon monoxide [GO:2001134] Also known as: down regulation of methane biosynthetic process from carbon monoxide, down-regulation of methane biosynthetic process from carbon monoxide, downregulation of methane biosynthetic process from carbon monoxide, inhibition of methane biosynthetic process from carbon monoxide Sources: GOC:TermGenie, GOC:mengo_curators Definition: Any process that stops, prevents or reduces the frequency, rate or extent of methane biosynthetic process from carbon monoxide.